positive regulation of penicillin metabolic process [GO:0033246] (biological process) Also known as: positive regulation of penicillin metabolism Definition: Any process that activates or increases the frequency, rate or extent of the chemical reactions and pathways involving any antibiotic that contains the condensed beta-lactamthiazolidine ring system. Subtypes: positive regulation of penicillin catabolic process [GO:0033249], GO:1900198 Relationships: is a type of positive regulation of amide metabolic process [GO:0034250]; is a type of regulation of sulfur metabolic process [GO:0042762]; is a type of regulation of secondary metabolic process [GO:0043455]; is a type of positive regulation of small molecule metabolic process [GO:0062013]; positively regulates penicillin metabolic process [GO:0042316] Sources: GOC:mah